peptide pheromone maturation [GO:0007323] (biological process) Definition: The generation of a mature, active peptide pheromone via processes unique to its processing and modification. An example of this process is found in Saccharomyces cerevisiae. Sources: GOC:elh Relationships: is_a protein maturation [GO:0051604] Also known as: pheromone processing